{
  "term_label": "intracellular sphingolipid homeostasis",
  "gene_symbol": "ORMDL3",
  "gene_name": "ORM1-like protein 3",
  "gene": "UniProtKB:Q8N138",
  "term_id": "GO:0090156"
}